{
  "gene_symbol": "TAS2R50",
  "gene": "UniProtKB:P59544",
  "gene_name": "Taste receptor type 2 member 50",
  "term_id": "GO:0033038",
  "term_label": "bitter taste receptor activity"
}